{
  "gene_name": "T-complex protein 1 subunit delta",
  "gene_symbol": "CCT4",
  "term_id": "GO:0006457",
  "gene": "UniProtKB:P50991",
  "term_label": "protein folding"
}